{
  "gene_name": "Immunoglobulin heavy diversity 5-12 (Fragment)",
  "gene": "UniProtKB:A0A0U1RQB9",
  "term_label": "Unknown molecular function",
  "gene_symbol": "IGHD5-12",
  "term_id": "UNKNOWN:0001"
}